{
  "gene": "UniProtKB:P16401",
  "gene_name": "Histone H1.5",
  "term_label": "negative regulation of DNA recombination",
  "term_id": "GO:0045910",
  "gene_symbol": "H1-5"
}